{
  "gene_name": "BPI fold-containing family B member 1",
  "gene_symbol": "BPIFB1",
  "term_label": "innate immune response in mucosa",
  "term_id": "GO:0002227",
  "gene": "UniProtKB:Q8TDL5"
}